{
  "gene": "UniProtKB:Q9BQE5",
  "gene_symbol": "APOL2",
  "gene_name": "Apolipoprotein L2",
  "term_label": "lipid binding",
  "term_id": "GO:0008289"
}